{
  "gene": "UniProtKB:Q7L099",
  "term_label": "neuronal cell body",
  "gene_symbol": "RUFY3",
  "term_id": "GO:0043025",
  "gene_name": "Protein RUFY3"
}